{
  "term_label": "excitatory extracellular ligand-gated monoatomic ion channel activity",
  "gene": "UniProtKB:Q9UGM1",
  "term_id": "GO:0005231",
  "gene_name": "Neuronal acetylcholine receptor subunit alpha-9",
  "gene_symbol": "CHRNA9"
}